{
  "gene_name": "Kinesin light chain 1",
  "gene_symbol": "KLC1",
  "term_label": "cytoplasm",
  "term_id": "GO:0005737",
  "gene": "UniProtKB:Q07866"
}